{
  "gene_name": "26S proteasome non-ATPase regulatory subunit 14",
  "gene": "UniProtKB:O00487",
  "term_label": "proteasome binding",
  "term_id": "GO:0070628",
  "gene_symbol": "PSMD14"
}